{
  "gene_symbol": "CLDN2",
  "gene": "UniProtKB:P57739",
  "gene_name": "Claudin-2",
  "term_id": "GO:0160187",
  "term_label": "paracellular tight junction channel activity"
}